{
  "gene_symbol": "SLIT2",
  "gene_name": "Slit homolog 2 protein",
  "term_label": "negative chemotaxis",
  "gene": "UniProtKB:O94813",
  "term_id": "GO:0050919"
}